{
  "term_label": "actin filament bundle",
  "term_id": "GO:0032432",
  "gene_symbol": "PLS1",
  "gene": "UniProtKB:Q14651",
  "gene_name": "Plastin-1"
}